sodium-translocating NADH:quinone reductase complex [GO:0160292] (cellular component) Also known as: Na(+)-translocating NADH-quinone reductase complex, Na+-NQR complex References: PMID:38955304 Relationships: is a type of protein-containing complex [GO:0032991] Definition: A bacterial protein complex consisting of six subunits, NqrABCDEF, encoded by the nqr operon, which catalyzes electron transfer from NADH to ubiquinone in the respiratory chain coupled with the transport of sodium ions from the cytoplasm to the periplasm.